{
  "gene": "UniProtKB:O14901",
  "gene_symbol": "KLF11",
  "term_id": "GO:0005634",
  "gene_name": "Krueppel-like factor 11",
  "term_label": "nucleus"
}